{
  "gene_name": "Angio-associated migratory cell protein",
  "term_label": "smooth muscle cell migration",
  "gene": "UniProtKB:Q13685",
  "term_id": "GO:0014909",
  "gene_symbol": "AAMP"
}